regulation of cell adhesion molecule production [GO:0060353] (biological process) Sources: GOC:BHF, GOC:rl Subtypes: negative regulation of cell adhesion molecule production [GO:0060354], GO:0060355 Definition: Any process that modulates the rate, frequency or extent of cell adhesion molecule production. Cell adhesion molecule production is the appearance of a cell adhesion molecule as a result of its biosynthesis or a decrease in its catabolism. Relationships: is a type of GO:0050794; regulates cell adhesion molecule production [GO:0060352]